vesicle transport along microtubule [GO:0047496] (biological process) Sources: GOC:ecd, GOC:rl Subtypes: minus-end-directed vesicle transport along microtubule [GO:0072382], plus-end-directed vesicle transport along microtubule [GO:0072383], GO:0099517, GO:1990048, retrograde neuronal dense core vesicle transport [GO:1990049] Regulation: regulated by regulation of vesicle transport along microtubule [GO:1901608]; negatively regulated by GO:1901609; positively regulated by positive regulation of vesicle transport along microtubule [GO:1901610] Relationships: is a type of GO:0072384; is a type of vesicle cytoskeletal trafficking [GO:0099518] Definition: The directed movement of a vesicle along a microtubule, mediated by motor proteins. This process begins with the attachment of a vesicle to a microtubule, and ends when the vesicle reaches its final destination. Also known as: microtubule-based vesicle localization